{
  "gene_name": "Tumor necrosis factor receptor type 1-associated DEATH domain protein",
  "gene": "UniProtKB:Q15628",
  "term_id": "GO:0005068",
  "gene_symbol": "TRADD",
  "term_label": "transmembrane receptor protein tyrosine kinase adaptor activity"
}